{
  "gene_name": "Glutaredoxin-1",
  "term_id": "UNKNOWN:0002",
  "gene": "UniProtKB:P35754",
  "term_label": "Unknown biological process",
  "gene_symbol": "GLRX"
}